{
  "term_id": "GO:0006352",
  "gene": "UniProtKB:Q92994",
  "gene_name": "Transcription factor IIIB 90 kDa subunit",
  "gene_symbol": "BRF1",
  "term_label": "DNA-templated transcription initiation"
}